{
  "gene_name": "X-ray repair cross-complementing protein 6",
  "gene_symbol": "XRCC6",
  "term_label": "telomeric DNA binding",
  "term_id": "GO:0042162",
  "gene": "UniProtKB:P12956"
}